{
  "gene": "UniProtKB:Q6PIF6",
  "term_label": "actin filament binding",
  "term_id": "GO:0051015",
  "gene_name": "Unconventional myosin-VIIb",
  "gene_symbol": "MYO7B"
}